{
  "gene": "UniProtKB:Q9H361",
  "gene_symbol": "PABPC3",
  "gene_name": "Polyadenylate-binding protein 3",
  "term_label": "poly(A) binding",
  "term_id": "GO:0008143"
}